{
  "term_id": "GO:0008582",
  "gene_symbol": "LIN7C",
  "gene": "UniProtKB:Q9NUP9",
  "term_label": "regulation of synaptic assembly at neuromuscular junction",
  "gene_name": "Protein lin-7 homolog C"
}